protein modification by small protein conjugation [GO:0032446] (biological process) Sources: GOC:mah Definition: A protein modification process in which one or more groups of a small protein, such as ubiquitin or a ubiquitin-like protein, are covalently attached to a target protein. Relationships: is a type of GO:0070647 Subtypes: GO:0016567, protein sumoylation [GO:0016925], GO:0032020, GO:0032447, protein neddylation [GO:0045116], protein pupylation [GO:0070490], protein ufmylation [GO:0071569]